positive regulation of siRNA processing [GO:1903705] (biological process) Relationships: is a type of positive regulation of metabolic process [GO:0009893]; is a type of regulation of siRNA processing [GO:0070921]; positively regulates siRNA processing [GO:0030422] Also known as: positive regulation of RNA interference, production of guide RNAs, positive regulation of RNA interference, production of siRNA, positive regulation of production of guide RNAs involved in RNA interference, positive regulation of production of siRNA involved in PTGS, positive regulation of production of siRNA involved in RNA interference, up regulation of RNA interference, production of guide RNAs, up regulation of RNA interference, production of siRNA, up regulation of production of guide RNAs involved in RNA interference, up regulation of production of siRNA involved in RNA interference, up-regulation of RNA interference, production of guide RNAs, up-regulation of RNA interference, production of siRNA, up-regulation of production of guide RNAs involved in RNA interference, up-regulation of production of siRNA involved in RNA interference, upregulation of RNA interference, production of guide RNAs, upregulation of RNA interference, production of siRNA, upregulation of production of guide RNAs involved in RNA interference, upregulation of production of siRNA involved in RNA interference, activation of RNA interference, production of guide RNAs, activation of RNA interference, production of siRNA, activation of production of guide RNAs involved in RNA interference, activation of production of siRNA involved in RNA interference, positive regulation of production of siRNA involved in post-transcriptional gene silencing by RNA, positive regulation of siRNA production Definition: Any process that activates or increases the frequency, rate or extent of siRNA processing. References: PMID:19701182 Sources: GOC:BHF, GOC:TermGenie, GOC:nc, GO_REF:0000058